{
  "term_id": "GO:0000172",
  "gene_symbol": "RPP25L",
  "term_label": "ribonuclease MRP complex",
  "gene": "UniProtKB:Q8N5L8",
  "gene_name": "Ribonuclease P protein subunit p25-like protein"
}